{
  "gene": "UniProtKB:Q96P09",
  "term_id": "GO:0051726",
  "gene_symbol": "BIRC8",
  "gene_name": "Baculoviral IAP repeat-containing protein 8",
  "term_label": "regulation of cell cycle"
}